positive regulation of fat cell differentiation [GO:0045600] (biological process) Relationships: is_a positive regulation of cell differentiation [GO:0045597]; is a type of regulation of fat cell differentiation [GO:0045598]; positively regulates fat cell differentiation [GO:0045444] Sources: GOC:go_curators Subtypes: GO:0090336 Definition: Any process that activates or increases the frequency, rate or extent of adipocyte differentiation. Also known as: positive regulation of adipocyte cell differentiation, positive regulation of adipocyte differentiation, up regulation of fat cell differentiation, up-regulation of fat cell differentiation, upregulation of fat cell differentiation, activation of fat cell differentiation, stimulation of fat cell differentiation